{
  "term_label": "Unknown molecular function",
  "gene": "UniProtKB:Q96H12",
  "gene_symbol": "MSANTD3",
  "term_id": "UNKNOWN:0001",
  "gene_name": "Myb_SANT-like DNA-binding domain-containing protein 3"
}